monocarboxylic acid transport [GO:0015718] (biological process) Definition: The directed movement of monocarboxylic acids into, out of or within a cell, or between cells, by means of some agent such as a transporter or pore. Sources: GOC:krc Relationships: is_a GO:0046942 Subtypes: GO:0006846, pyruvate transport [GO:0006848], phosphoenolpyruvate transport [GO:0015714], allantoate transport [GO:0015719], bile acid and bile salt transport [GO:0015721], formate transport [GO:0015724], lactate transport [GO:0015727], shikimate transmembrane transport [GO:0015733], uronic acid transmembrane transport [GO:0015735], biotin transport [GO:0015878], creatine transmembrane transport [GO:0015881], pantothenate transmembrane transport [GO:0015887], fatty acid transport [GO:0015908], GO:0032782, hydroxyectoine transmembrane transport [GO:0033308], GO:0034659, aldonate transmembrane transport [GO:0042873], benzoate transport [GO:0042919], 3-hydroxyphenylpropionic acid transmembrane transport [GO:0042920], 2-keto-3-deoxygluconate transmembrane transport [GO:0046411], GO:0051470, abscisic acid transport [GO:0080168], 5-aminolevulinic acid import across plasma membrane [GO:0140484], 4-hydroxyphenylacetate transport [GO:1900754], glycolate transport [GO:1900866], dethiobiotin import across plasma membrane [GO:1905136], nicotinate transport [GO:2001142]